apocrine secretion [GO:0160022] (BP) Also known as: secretion by cell decapitation, secretion by membrane budding References: PMID:25960390 Definition: The controlled release of a substance by a cell or a tissue by discharging a portion of the secreting cell when intracellular components are freed into a lumen through the shedding of whole pieces of the cytoplasm. Relationships: is a type of secretion [GO:0046903]